{
  "term_id": "GO:0005737",
  "gene_symbol": "PKP2",
  "term_label": "cytoplasm",
  "gene_name": "Plakophilin-2",
  "gene": "UniProtKB:Q99959"
}